negative regulation of asexual reproduction [GO:1903665] (biological process) Definition: Any process that stops, prevents or reduces the frequency, rate or extent of asexual reproduction. References: PMID:24390142 Sources: GOC:TermGenie, GO_REF:0000058 Also known as: down regulation of asexual reproduction, down-regulation of asexual reproduction, downregulation of asexual reproduction, inhibition of asexual reproduction Relationships: is a type of regulation of asexual reproduction [GO:1903664]; is a type of negative regulation of reproductive process [GO:2000242]; negatively regulates GO:0019954 Subtypes: negative regulation of asexual sporulation resulting in formation of a cellular spore [GO:0043944], negative regulation of cell budding [GO:0045781], negative regulation of conidium formation [GO:0075308], negative regulation of oomycete sporangium development [GO:0075324]